{
  "gene_symbol": "TBX2",
  "gene": "UniProtKB:Q13207",
  "term_label": "chromatin",
  "gene_name": "T-box transcription factor TBX2",
  "term_id": "GO:0000785"
}